D-glucuronate catabolic process to D-xylulose 5-phosphate [GO:0019640] (biological process) Definition: The chemical reactions and pathways resulting in the breakdown of D-glucuronate into D-xylulose 5-phosphate. References: PMID:27189775 Sources: GOC:go_curators Also known as: glucuronate breakdown to xylulose 5-phosphate, glucuronate catabolic process to xylulose 5-phosphate, glucuronate degradation to xylulose 5-phosphate Relationships: is a type of GO:0042840; is a type of D-xylulose 5-phosphate metabolic process [GO:0051167]